{
  "gene_name": "Caldesmon",
  "term_id": "GO:0017022",
  "gene": "UniProtKB:Q05682",
  "term_label": "myosin binding",
  "gene_symbol": "CALD1"
}